regulation of potassium ion import [GO:1903286] (biological process) Subtypes: GO:1903287, positive regulation of potassium ion import across plasma membrane [GO:1903288] References: PMID:10636900 Sources: GOC:BHF, GOC:TermGenie, GOC:mtg_cardiac_conduct_nov11, GOC:rl, GO_REF:0000058 Definition: Any process that modulates the frequency, rate or extent of potassium ion import. Also known as: regulation of potassium import, regulation of potassium ion uptake Relationships: is a type of regulation of potassium ion transmembrane transport [GO:1901379]; RO_0002211 GO:1990573